{
  "gene_name": "Keratin, type II cytoskeletal 6B",
  "gene_symbol": "KRT6B",
  "term_id": "GO:0045095",
  "gene": "UniProtKB:P04259",
  "term_label": "keratin filament"
}